{
  "gene": "UniProtKB:Q15139",
  "term_label": "phospholipase C-activating G protein-coupled receptor signaling pathway",
  "gene_name": "Serine_threonine-protein kinase D1",
  "term_id": "GO:0007200",
  "gene_symbol": "PRKD1"
}